L-arginine biosynthetic process via N-acetyl-L-citrulline [GO:0170067] (biological process) Also known as: arginine biosynthesis via N-acetyl intermediates, arginine biosynthesis, N-acetylated pathway Relationships: is a type of L-arginine biosynthetic process [GO:0006526] Definition: The chemical reactions and pathways resulting in the formation of arginine (2-amino-5-guanidinopentanoic acid) via the intermediate compound N-acetyl-L-citrulline. References: PMID:16585758